{
  "gene_symbol": "SLC26A6",
  "term_id": "GO:0140900",
  "term_label": "chloride:bicarbonate antiporter activity",
  "gene_name": "Solute carrier family 26 member 6",
  "gene": "UniProtKB:Q9BXS9"
}